{
  "gene": "UniProtKB:Q8NBH2",
  "gene_name": "Kyphoscoliosis peptidase",
  "term_id": "UNKNOWN:0001",
  "gene_symbol": "KY",
  "term_label": "Unknown molecular function"
}